{
  "gene_name": "E3 ubiquitin-protein ligase BRE1B",
  "gene_symbol": "RNF40",
  "term_id": "GO:0033503",
  "gene": "UniProtKB:O75150",
  "term_label": "HULC complex"
}